7,8-didemethyl-8-hydroxy-5-deazariboflavin synthase activity [GO:0044689] (molecular function) Also known as: FO synthase Definition: Catalysis of the reaction: 5-amino-5-(4-hydroxybenzyl)-6-(D-ribitylimino)-5,6-dihydrouracil + S-adenosyl-L-methionine = 5'-deoxyadenosine + 7,8-didemethyl-8-hydroxy-5-deazariboflavin + H+ + L-methionine + NH4+. References: PMID:14593448 Sources: RHEA:55204 Relationships: is a type of GO:0016841